{
  "gene_symbol": "CHD1L",
  "gene_name": "Chromodomain-helicase-DNA-binding protein 1-like",
  "gene": "UniProtKB:Q86WJ1",
  "term_id": "GO:0000166",
  "term_label": "nucleotide binding"
}